{
  "gene_symbol": "GALNT4",
  "term_id": "UNKNOWN:0003",
  "gene": "UniProtKB:Q8N4A0",
  "term_label": "Unknown cellular component",
  "gene_name": "Polypeptide N-acetylgalactosaminyltransferase 4"
}